{
  "term_label": "proton-transporting ATP synthase activity, rotational mechanism",
  "gene_name": "ATP synthase subunit d, mitochondrial",
  "gene": "UniProtKB:O75947",
  "term_id": "GO:0046933",
  "gene_symbol": "ATP5PD"
}